regulation of anther dehiscence [GO:0120194] (biological process) References: PMID:30911018 Sources: GOC:lr Relationships: is a type of regulation of reproductive process [GO:2000241]; regulates anther dehiscence [GO:0009901] Subtypes: positive regulation of anther dehiscence [GO:0120195], negative regulation of anther dehiscence [GO:0120196] Definition: Any process involved in the dehiscence of an anther to release the pollen grains contained within it.